{
  "gene_name": "Ankyrin repeat domain-containing protein 36C",
  "gene_symbol": "ANKRD36C",
  "gene": "UniProtKB:Q5JPF3",
  "term_label": "Unknown biological process",
  "term_id": "UNKNOWN:0002"
}